{
  "gene": "UniProtKB:Q6ZNJ1",
  "gene_symbol": "NBEAL2",
  "gene_name": "Neurobeachin-like protein 2",
  "term_label": "membrane",
  "term_id": "GO:0016020"
}